{
  "gene_name": "Calcium load-activated calcium channel",
  "gene": "UniProtKB:Q9UM00",
  "gene_symbol": "TMCO1",
  "term_label": "calcium channel activity",
  "term_id": "GO:0005262"
}